{
  "term_label": "[heparan sulfate]-glucosamine 3-sulfotransferase activity",
  "gene": "UniProtKB:Q8IZT8",
  "term_id": "GO:0008467",
  "gene_symbol": "HS3ST5",
  "gene_name": "Heparan sulfate glucosamine 3-O-sulfotransferase 5"
}